{
  "gene_name": "E3 ubiquitin-protein ligase RNF128",
  "gene_symbol": "RNF128",
  "gene": "UniProtKB:Q8TEB7",
  "term_label": "late endosome",
  "term_id": "GO:0005770"
}